{
  "gene_name": "Actin-like protein 8",
  "term_id": "GO:0035267",
  "gene": "UniProtKB:Q9H568",
  "term_label": "NuA4 histone acetyltransferase complex",
  "gene_symbol": "ACTL8"
}